{
  "gene_name": "Cyclic GMP-AMP synthase",
  "term_id": "GO:0006974",
  "gene_symbol": "CGAS",
  "gene": "UniProtKB:Q8N884",
  "term_label": "DNA damage response"
}